{
  "term_id": "GO:0005829",
  "gene_symbol": "PGK1",
  "term_label": "cytosol",
  "gene": "UniProtKB:P00558",
  "gene_name": "Phosphoglycerate kinase 1"
}